{
  "gene_name": "Histone H3.1",
  "gene_symbol": "H3C12",
  "gene": "UniProtKB:P68431",
  "term_label": "heterochromatin formation",
  "term_id": "GO:0031507"
}